{
  "term_label": "RNA polymerase II transcription regulatory region sequence-specific DNA binding",
  "gene": "UniProtKB:Q8TC21",
  "gene_symbol": "ZNF596",
  "term_id": "GO:0000977",
  "gene_name": "Zinc finger protein 596"
}